interleukin-33 binding [GO:0002113] (molecular function) Also known as: IL-33 binding Relationships: is a type of GO:0019955 Definition: Binding to interleukin-33. Sources: GOC:hjd